{
  "gene_symbol": "MFAP4",
  "gene": "UniProtKB:P55083",
  "term_id": "GO:0005615",
  "gene_name": "Microfibril-associated glycoprotein 4",
  "term_label": "extracellular space"
}